{
  "gene_name": "Late cornified envelope protein 7A",
  "gene_symbol": "LCE7A",
  "term_label": "Unknown molecular function",
  "gene": "UniProtKB:P0DV60",
  "term_id": "UNKNOWN:0001"
}